{
  "term_id": "GO:0015459",
  "gene": "UniProtKB:Q13303",
  "term_label": "potassium channel regulator activity",
  "gene_symbol": "KCNAB2",
  "gene_name": "Voltage-gated potassium channel subunit beta-2"
}